{
  "gene_symbol": "ELOVL1",
  "gene": "UniProtKB:Q9BW60",
  "term_label": "very long-chain fatty acid biosynthetic process",
  "gene_name": "Elongation of very long chain fatty acids protein 1",
  "term_id": "GO:0042761"
}